endosomal scaffold complex [GO:0032969] (cellular component) Relationships: is a type of membrane protein complex [GO:0098796]; is part of late endosome membrane [GO:0031902] Also known as: MP1-p14 scaffolding complex, endosomal adaptor complex Definition: A protein complex that contains MAPKSP1 (MP1, Map2k1ip1) and ROBLD3 (p14, Mapbpip), is anchored to late endosomes, and is involved in selective activation of the ERK1 in ERK/MAPK signaling. References: PMID:15263099, PMID:16227978, PMID:17496910